protein catabolic process, modulating synaptic transmission [GO:0099546] (biological process) References: PMID:23083742 Sources: GOC:dos Relationships: is a type of protein catabolic process at synapse [GO:0140246]; regulates GO:0007268 Definition: Any protein degradation process, occurring at a presynapse, that regulates synaptic transmission. Note: Note that this term was created for the SynGO project, and will be obsoleted when the SynGO annotations are made in Noctua.